{
  "term_label": "small GTPase binding",
  "gene_symbol": "RANGRF",
  "gene": "UniProtKB:Q9HD47",
  "gene_name": "Ran guanine nucleotide release factor",
  "term_id": "GO:0031267"
}